{
  "gene": "UniProtKB:Q9P225",
  "gene_symbol": "DNAH2",
  "term_id": "GO:0008569",
  "gene_name": "Dynein axonemal heavy chain 2",
  "term_label": "minus-end-directed microtubule motor activity"
}